alanine transport [GO:0032328] (biological process) Subtypes: L-alanine transport [GO:0015808], D-alanine transmembrane transport [GO:0042941] Relationships: is a type of GO:0015695; is a type of neutral amino acid transport [GO:0015804]; is_a carboxylic acid transport [GO:0046942]; is a type of nitrogen compound transport [GO:0071705] Definition: The directed movement of alanine, 2-aminopropanoic acid, into, out of or within a cell, or between cells, by means of some agent such as a transporter or pore. Sources: GOC:mah